regulation of ERK5 cascade [GO:0070376] (biological process) Sources: GOC:add, ISBN:0121245462, ISBN:0896039986 Subtypes: negative regulation of ERK5 cascade [GO:0070377], positive regulation of ERK5 cascade [GO:0070378] Definition: Any process that modulates the frequency, rate or extent of signal transduction mediated by the ERK5 cascade. Relationships: is a type of regulation of MAPK cascade [GO:0043408]; regulates ERK5 cascade [GO:0070375] Also known as: regulation of BMK cascade, regulation of BMK signaling pathway, regulation of BMK signalling pathway, regulation of BMK1 cascade, regulation of ERK5 signaling pathway, regulation of MAPK7 cascade